{
  "gene_symbol": "KIF3C",
  "gene": "UniProtKB:O14782",
  "term_id": "GO:0005737",
  "term_label": "cytoplasm",
  "gene_name": "Kinesin-like protein KIF3C"
}